{
  "gene_symbol": "OR51G2",
  "gene_name": "Olfactory receptor 51G2",
  "term_id": "GO:0004984",
  "gene": "UniProtKB:Q8NGK0",
  "term_label": "olfactory receptor activity"
}